border follicle cell delamination [GO:0030709] (biological process) Also known as: border cell delamination References: PMID:10822261 Relationships: is a type of GO:0060232; is part of follicle cell of egg chamber development [GO:0030707] Regulation: regulated by GO:0030710; positively regulated by positive regulation of border follicle cell delamination [GO:0030711]; negatively regulated by negative regulation of border follicle cell delamination [GO:0030712] Definition: The delamination process that results in the splitting off of border cells from the anterior epithelium, prior to border cell migration.